{
  "term_id": "UNKNOWN:0001",
  "gene_name": "Nucleoporin SEH1",
  "gene": "UniProtKB:Q96EE3",
  "gene_symbol": "SEH1L",
  "term_label": "Unknown molecular function"
}